Sertoli cell fate commitment [GO:0060010] (biological process) Relationships: is_a GO:0003006; is a type of GO:0072148; is part of Sertoli cell differentiation [GO:0060008] Definition: The process in which the cellular identity of Sertoli cells is acquired and determined. Sources: GOC:dph